{
  "gene": "UniProtKB:Q15173",
  "term_label": "Unknown biological process",
  "term_id": "UNKNOWN:0002",
  "gene_symbol": "PPP2R5B",
  "gene_name": "Serine_threonine-protein phosphatase 2A 56 kDa regulatory subunit beta isoform"
}